melibiose:sodium symporter activity [GO:0043887] (molecular function) References: PMID:1970646 Definition: Enables the transfer of a solute or solutes from one side of a membrane to the other according to the reaction: melibiose(out) + Na+(out) = melibiose(in) + Na+(in). Also known as: melibiose permease, Na+ (Li+)/melibiose symporter activity, Na+-melibiose symporter activity, Na+/melibiose symporter activity, Na+:melibiose symporter activity, melibiose-Na+ symporter activity, melibiose-sodium symporter activity, melibiose/Na+ symporter activity, melibiose/sodium symporter activity, melibiose:Na+ symporter activity, sodium-melibiose symporter activity, sodium/melibiose symporter activity, sodium:melibiose symporter activity, MelB, melibiose carrier protein, thiomethylgalactoside permease II Relationships: is a type of solute:sodium symporter activity [GO:0015370]; is a type of melibiose:monoatomic cation symporter activity [GO:0015487]